{
  "gene_symbol": "CERKL",
  "term_id": "GO:0006665",
  "term_label": "sphingolipid metabolic process",
  "gene_name": "Ceramide kinase-like protein",
  "gene": "UniProtKB:Q49MI3"
}